negative regulation of neutrophil mediated killing of gram-negative bacterium [GO:0070957] (biological process) Sources: GOC:add, GOC:mah Also known as: down regulation of neutrophil mediated killing of gram-negative bacterium, down-regulation of neutrophil mediated killing of gram-negative bacterium, downregulation of neutrophil mediated killing of gram-negative bacterium, inhibition of neutrophil mediated killing of gram-negative bacterium Relationships: is a type of GO:0070951; is a type of negative regulation of neutrophil mediated killing of bacterium [GO:0070956]; negatively regulates GO:0070945 Definition: Any process that decreases the frequency, rate or extent of the directed killing of a gram-negative bacterium by a neutrophil.